{
  "gene_name": "NADH dehydrogenase [ubiquinone] 1 alpha subcomplex subunit 4-like 2",
  "term_label": "Unknown molecular function",
  "gene_symbol": "NDUFA4L2",
  "term_id": "UNKNOWN:0001",
  "gene": "UniProtKB:Q9NRX3"
}